{
  "gene_name": "Eukaryotic translation initiation factor 1A, X-chromosomal",
  "gene_symbol": "EIF1AX",
  "term_label": "translational initiation",
  "gene": "UniProtKB:P47813",
  "term_id": "GO:0006413"
}